{
  "gene_name": "Protein odd-skipped-related 2",
  "gene_symbol": "OSR2",
  "term_id": "GO:0007389",
  "term_label": "pattern specification process",
  "gene": "UniProtKB:Q8N2R0"
}